ER body organization [GO:0080119] (biological process) Also known as: ER body organisation, endoplasmic reticulum body organization, ER body organization and biogenesis, endoplasmic reticulum body organization and biogenesis Definition: A process that is carried out at the cellular level which results in the formation of ER (endoplasmic reticulum) body. ER body is a compartment found in plant cells that is derived from the ER. The structures have a characteristic shape and size (10 mm long and 0.5 mm wide) and are surrounded with ribosomes. They have been found in Arabidopsis thaliana and related Brassicaceae species. Relationships: is a type of organelle organization [GO:0006996] References: PMID:18780803, PMID:19147648